{
  "gene_symbol": "TRAJ25",
  "term_id": "UNKNOWN:0003",
  "gene": "UniProtKB:A0A075B6Z8",
  "term_label": "Unknown cellular component",
  "gene_name": "T cell receptor alpha joining 25 (non-functional) (Fragment)"
}